regulation of endothelial cell chemotaxis to vascular endothelial growth factor [GO:1904857] (biological process) References: PMID:21885851 Sources: GOC:BHF, GOC:BHF_miRNA, GOC:TermGenie, GOC:rph, GO_REF:0000058 Relationships: is a type of regulation of cell migration [GO:0030334]; is a type of regulation of chemotaxis [GO:0050920]; is a type of regulation of cellular response to vascular endothelial growth factor stimulus [GO:1902547]; regulates endothelial cell chemotaxis to vascular endothelial growth factor [GO:0090668] Subtypes: negative regulation of endothelial cell chemotaxis to vascular endothelial growth factor [GO:1904858], positive regulation of endothelial cell chemotaxis to vascular endothelial growth factor [GO:1904859] Definition: Any process that modulates the frequency, rate or extent of endothelial cell chemotaxis to vascular endothelial growth factor.